positive regulation of neuron maturation [GO:0014042] (biological process) Subtypes: positive regulation of neuron remodeling [GO:1904801] Relationships: is a type of GO:0014041; is a type of GO:1903431; RO_0002213 neuron maturation [GO:0042551] Sources: GOC:ef Definition: Any process that activates or increases the frequency, rate or extent of neuron maturation. Also known as: up regulation of neuron maturation, up-regulation of neuron maturation, upregulation of neuron maturation, activation of neuron maturation, stimulation of neuron maturation